{
  "gene_symbol": "Q8NAQ8",
  "gene_name": "Putative uncharacterized protein FLJ34945",
  "term_label": "Unknown molecular function",
  "term_id": "UNKNOWN:0001",
  "gene": "UniProtKB:Q8NAQ8"
}